{
  "term_id": "GO:0005737",
  "gene": "UniProtKB:Q9BZK3",
  "gene_symbol": "NACA4P",
  "gene_name": "Putative nascent polypeptide-associated complex subunit alpha-like protein",
  "term_label": "cytoplasm"
}